low-affinity zinc ion transmembrane transporter activity [GO:0000007] (molecular function) Relationships: is a type of zinc ion transmembrane transporter activity [GO:0005385] Sources: GOC:mtg_transport, ISBN:0815340729 Definition: Enables the transfer of a solute or solutes from one side of a membrane to the other according to the reaction: Zn2+ = Zn2+, probably powered by proton motive force. In low-affinity transport the transporter is able to bind the solute only if it is present at very high concentrations.